{
  "term_id": "GO:0004984",
  "gene_name": "Olfactory receptor 7D2",
  "gene_symbol": "OR7D2",
  "gene": "UniProtKB:Q96RA2",
  "term_label": "olfactory receptor activity"
}